glycine biosynthetic process [GO:0006545] (biological process) Also known as: glycine anabolism, glycine biosynthesis, glycine formation, glycine synthesis Subtypes: glycine biosynthetic process from serine [GO:0019264], glycine biosynthetic process, by transamination of glyoxylate [GO:0019265], L-threonine catabolic process to glycine [GO:0019518] Relationships: is a type of glycine metabolic process [GO:0006544]; is a type of GO:0009070; is a type of proteinogenic amino acid biosynthetic process [GO:0170038] Definition: The chemical reactions and pathways resulting in the formation of glycine, aminoethanoic acid. Sources: GOC:go_curators